{
  "gene_symbol": "KRT16",
  "gene_name": "Keratin, type I cytoskeletal 16",
  "gene": "UniProtKB:P08779",
  "term_id": "GO:0030280",
  "term_label": "structural constituent of skin epidermis"
}